{
  "gene_symbol": "CEPT1",
  "gene": "UniProtKB:Q9Y6K0",
  "term_id": "GO:0005789",
  "gene_name": "Choline_ethanolaminephosphotransferase 1",
  "term_label": "endoplasmic reticulum membrane"
}